{
  "term_label": "cytoskeleton",
  "gene": "UniProtKB:Q494U1",
  "term_id": "GO:0005856",
  "gene_name": "Pleckstrin homology domain-containing family N member 1",
  "gene_symbol": "PLEKHN1"
}